histone H4K12 acetyltransferase activity [GO:0043997] (MF) Relationships: is a type of GO:0010485 Also known as: histone H4-K12 acetyltransferase activity, histone acetylase activity (H4-K12 specific), histone acetyltransferase activity (H4-K12 specific), histone lysine N-acetyltransferase activity (H4-K12 specific) Note: Note that the residue position corresponds to the canonical human H4 histone (UniProtKB:P02309); this residue is conserved across all eukaryotes. Note that the initiation methionine is cleaved, so the first residue is S1. Definition: Catalysis of the reaction: acetyl-CoA + histone H4 L-lysine (position 12) = CoA + histone H4 N6-acetyl-L-lysine (position 12). References: PMID:18552846, PMID:19056256